{
  "gene_symbol": "NEDD1",
  "term_label": "centrosome",
  "gene_name": "Protein NEDD1",
  "gene": "UniProtKB:Q8NHV4",
  "term_id": "GO:0005813"
}